regulation of filamentous growth of a population of unicellular organisms [GO:1900428] (biological process) Relationships: is a type of regulation of filamentous growth [GO:0010570]; regulates filamentous growth of a population of unicellular organisms [GO:0044182] Subtypes: regulation of growth of unicellular organism as a thread of attached cells [GO:0070784], GO:1900429, positive regulation of filamentous growth of a population of unicellular organisms [GO:1900430], regulation of filamentous growth of a population of unicellular organisms in response to heat [GO:1900431], GO:1900434, regulation of filamentous growth of a population of unicellular organisms in response to chemical stimulus [GO:1900437], regulation of filamentous growth of a population of unicellular organisms in response to biotic stimulus [GO:1900443], regulation of filamentous growth of a population of unicellular organisms in response to pH [GO:1900741] Sources: GOC:TermGenie, GOC:di Definition: Any process that modulates the frequency, rate or extent of filamentous growth of a population of unicellular organisms.